ergosterol metabolic process [GO:0008204] (biological process) Definition: The chemical reactions and pathways involving ergosterol, (22E)-ergosta-5,7,22-trien-3-beta-ol, a sterol found in ergot, yeast and moulds. It is the most important of the D provitamins and is converted to vitamin D2 on irradiation with UV light. Sources: ISBN:0198506732 Also known as: ergosterol metabolism Relationships: is a type of sterol metabolic process [GO:0016125]; is a type of secondary alcohol metabolic process [GO:1902652] Subtypes: ergosterol biosynthetic process [GO:0006696]